{
  "term_id": "UNKNOWN:0003",
  "term_label": "Unknown cellular component",
  "gene_name": "DEP domain-containing protein 1B",
  "gene": "UniProtKB:Q8WUY9",
  "gene_symbol": "DEPDC1B"
}